{
  "gene_symbol": "PDXDC1",
  "term_id": "UNKNOWN:0002",
  "term_label": "Unknown biological process",
  "gene_name": "Pyridoxal-dependent decarboxylase domain-containing protein 1",
  "gene": "UniProtKB:Q6P996"
}